Fc receptor-mediated immune complex endocytosis [GO:0160006] (biological process) Relationships: is a type of receptor-mediated endocytosis [GO:0006898] Also known as: Ig-complexed antigen endocytosis via Fc receptor, antigen-antibody immune complex uptake via Fc receptor, Fc receptor-mediated immune complex internalization References: PMID:28389502, PMID:9143687, PMID:9463401 Definition: An endocytosis process mediated by the Fc receptor for the purpose of delivery of antigen-bound immunoglobulin to an intracellular compartment where the antigen can be processed and loaded onto MHC molecules. This process selectively targets antigens for presentation by MHC class II or cross-presentation by MHC class I.